{
  "gene_symbol": "KIAA0232",
  "term_id": "UNKNOWN:0001",
  "gene": "UniProtKB:Q92628",
  "gene_name": "Uncharacterized protein KIAA0232",
  "term_label": "Unknown molecular function"
}